{
  "gene_symbol": "ARHGAP1",
  "term_label": "negative regulation of endocytic recycling",
  "gene": "UniProtKB:Q07960",
  "gene_name": "Rho GTPase-activating protein 1",
  "term_id": "GO:2001136"
}